{
  "gene": "UniProtKB:Q96NC0",
  "gene_name": "Zinc finger matrin-type protein 2",
  "term_id": "GO:0000398",
  "term_label": "mRNA splicing, via spliceosome",
  "gene_symbol": "ZMAT2"
}